{
  "term_id": "GO:0045087",
  "gene": "UniProtKB:Q8N688",
  "gene_symbol": "DEFB123",
  "term_label": "innate immune response",
  "gene_name": "Beta-defensin 123"
}